{
  "gene_name": "Rho GDP-dissociation inhibitor 1",
  "gene_symbol": "ARHGDIA",
  "term_label": "Rho protein signal transduction",
  "term_id": "GO:0007266",
  "gene": "UniProtKB:P52565"
}